{
  "term_label": "serine-type peptidase activity",
  "term_id": "GO:0008236",
  "gene_name": "Serine protease FAM111B",
  "gene_symbol": "FAM111B",
  "gene": "UniProtKB:Q6SJ93"
}